regulation of intraciliary retrograde transport [GO:1905799] (biological process) References: PMID:27930654 Sources: GOC:TermGenie, GO_REF:0000058 Subtypes: negative regulation of intraciliary retrograde transport [GO:1905800], GO:1905801 Also known as: regulation of intraflagellar retrograde transport Relationships: is a type of regulation of intracellular transport [GO:0032386]; is a type of regulation of microtubule-based movement [GO:0060632]; RO_0002211 intraciliary retrograde transport [GO:0035721] Definition: Any process that modulates the frequency, rate or extent of intraciliary retrograde transport.